{
  "gene_name": "Zinc finger protein 749",
  "term_label": "RNA polymerase II transcription regulatory region sequence-specific DNA binding",
  "term_id": "GO:0000977",
  "gene_symbol": "ZNF749",
  "gene": "UniProtKB:O43361"
}